{
  "term_label": "histone binding",
  "gene_name": "Testis-specific Y-encoded-like protein 5",
  "gene": "UniProtKB:Q86VY4",
  "term_id": "GO:0042393",
  "gene_symbol": "TSPYL5"
}